regulation of maltohexaose transport [GO:1900312] (biological process) Sources: GOC:TermGenie, GOC:mengo_curators Subtypes: negative regulation of maltohexaose transport [GO:1900313], GO:1900314 Definition: Any process that modulates the frequency, rate or extent of maltohexaose transport. Relationships: is a type of regulation of hexasaccharide transport [GO:1900297]; regulates maltohexaose transport [GO:2001103]